{
  "term_label": "heme binding",
  "gene_symbol": "CYP2D6",
  "term_id": "GO:0020037",
  "gene_name": "Cytochrome P450 2D6",
  "gene": "UniProtKB:P10635"
}